{
  "term_id": "UNKNOWN:0001",
  "gene_symbol": "TPD52L3",
  "gene_name": "Tumor protein D55",
  "term_label": "Unknown molecular function",
  "gene": "UniProtKB:Q96J77"
}